{
  "gene_symbol": "SHMT2",
  "gene_name": "Serine hydroxymethyltransferase, mitochondrial",
  "gene": "UniProtKB:P34897",
  "term_id": "GO:0005739",
  "term_label": "mitochondrion"
}